regulation of extraocular skeletal muscle development [GO:0014725] (biological process) Definition: Any process that modulates the frequency, rate or extent of extraocular skeletal muscle development. Extraocular skeletal muscle development is the process whose specific outcome is the progression of the extraocular skeletal muscle over time, from its formation to the mature structure. The extraocular muscle is derived from cranial mesoderm and controls eye movements. The muscle begins its development with the differentiation of the muscle cells and ends with the mature muscle. Subtypes: negative regulation of extraocular skeletal muscle development [GO:0014726], positive regulation of extraocular skeletal muscle development [GO:0014727] Relationships: is a type of regulation of skeletal muscle tissue development [GO:0048641]; regulates extraocular skeletal muscle development [GO:0002074] Sources: GOC:mtg_muscle